cellular response to epinephrine stimulus [GO:0071872] (biological process) Relationships: is a type of GO:0070887; is a type of response to epinephrine [GO:0071871] Also known as: cellular response to adrenaline stimulus Definition: Any process that results in a change in state or activity of a cell (in terms of movement, secretion, enzyme production, gene expression, etc.) as a result of an epinephrine stimulus. Epinephrine is a catecholamine that has the formula C9H13NO3; it is secreted by the adrenal medulla to act as a hormone, and released by certain neurons to act as a neurotransmitter active in the central nervous system. Note: Note that epinephrine and norepinephrine are ligands for the same receptors, and there are multiple adrenergic receptors. Sources: GOC:BHF, GOC:mah